{
  "gene_name": "Cytochrome P450 4F3",
  "term_id": "GO:0042361",
  "gene_symbol": "CYP4F3",
  "gene": "UniProtKB:Q08477",
  "term_label": "menaquinone catabolic process"
}